imaginal disc-derived wing hair elongation [GO:0035319] (biological process) Also known as: wing hair elongation, wing prehair extension References: PMID:11832234 Sources: GOC:mtg_sensu Definition: Growth of a prehair in the approximately 10 hour period following its emergence from an epidermal cell in an imaginal disc-derived wing. Prehair elongation is guided and/or driven by the polymerization of actin filaments and the orderly crosslinking of filaments into bundles. Relationships: is a type of post-embryonic animal morphogenesis [GO:0009886]; is a type of cell projection morphogenesis [GO:0048858]; is part of imaginal disc-derived wing hair organization [GO:0035317]